box H/ACA sno(s)RNA metabolic process [GO:0033979] (biological process) Relationships: is a type of sno(s)RNA metabolic process [GO:0016074] Also known as: box H/ACA sRNA metabolic process, box H/ACA snoRNA metabolic process Definition: The chemical reactions and pathways involving box H/ACA type small nucleolar RNA. Sources: GOC:krc, GOC:mah Subtypes: box H/ACA sno(s)RNA processing [GO:0034964]